{
  "gene": "UniProtKB:A6NFT4",
  "term_id": "UNKNOWN:0001",
  "gene_symbol": "CFAP73",
  "term_label": "Unknown molecular function",
  "gene_name": "Cilia- and flagella-associated protein 73"
}